clathrin-coated vesicle membrane [GO:0030665] (cellular component) Sources: GOC:mah Also known as: clathrin coated vesicle membrane Relationships: is a type of coated vesicle membrane [GO:0030662]; is part of GO:0030136 Subtypes: trans-Golgi network transport vesicle membrane [GO:0012510], clathrin-coated endocytic vesicle membrane [GO:0030669], clathrin-sculpted acetylcholine transport vesicle membrane [GO:0060201], GO:0060203, GO:0061202, clathrin-sculpted monoamine transport vesicle membrane [GO:0070083] Definition: The lipid bilayer surrounding a clathrin-coated vesicle.